{
  "term_id": "GO:0005737",
  "gene_name": "A-kinase anchor protein 11",
  "term_label": "cytoplasm",
  "gene_symbol": "AKAP11",
  "gene": "UniProtKB:Q9UKA4"
}